L-proline betaine catabolic process [GO:0019504] (biological process) References: PMID:10689197, PMID:1804402, PMID:24520058 Also known as: stachydrine breakdown, stachydrine catabolic process, stachydrine catabolism, stachydrine degradation Relationships: is a type of amino-acid betaine catabolic process [GO:0006579]; is_a GO:0009822; is a type of L-amino acid catabolic process [GO:0170035]; is a type of GO:0170044 Definition: The chemical reactions and pathways resulting in the breakdown of stachydrine, N-methylproline methylbetaine, the betaine derivative of L-proline.